{
  "gene_symbol": "SLC12A7",
  "gene": "UniProtKB:Q9Y666",
  "term_label": "potassium ion import across plasma membrane",
  "gene_name": "Solute carrier family 12 member 7",
  "term_id": "GO:1990573"
}